{
  "gene_name": "Vesicular acetylcholine transporter",
  "term_id": "GO:0005277",
  "term_label": "acetylcholine transmembrane transporter activity",
  "gene": "UniProtKB:Q16572",
  "gene_symbol": "SLC18A3"
}